phosphopentomutase activity [GO:0008973] (molecular function) Definition: Catalysis of the reaction: D-ribose 1-phosphate = D-ribose 5-phosphate. Also converts 2-deoxy-alpha-D-ribose 1-phosphate into 2-deoxy-D-ribose 5-phosphate. Relationships: is a type of intramolecular phosphotransferase activity [GO:0016868] Sources: EC:5.4.2.7 Also known as: D-ribose 1,5-phosphomutase activity, alpha-D-glucose-1,6-bisphosphate:deoxy-D-ribose-1-phosphate phosphotransferase activity, alpha-D-ribose 1,5-phosphomutase activity, deoxyribomutase activity, deoxyribose phosphomutase activity, phosphodeoxyribomutase activity, phosphoribomutase activity